{
  "gene_name": "Palmitoyl-protein thioesterase ABHD10, mitochondrial",
  "term_label": "mitochondrion",
  "gene_symbol": "ABHD10",
  "term_id": "GO:0005739",
  "gene": "UniProtKB:Q9NUJ1"
}